{
  "gene_name": "U4_U6.U5 tri-snRNP-associated protein 1",
  "term_label": "U4/U6 x U5 tri-snRNP complex",
  "gene_symbol": "SART1",
  "term_id": "GO:0046540",
  "gene": "UniProtKB:O43290"
}